{
  "gene": "UniProtKB:P0CJ74",
  "term_label": "Unknown cellular component",
  "gene_symbol": "MTRNR2L7",
  "gene_name": "Humanin-like 7",
  "term_id": "UNKNOWN:0003"
}